{
  "term_label": "Unknown molecular function",
  "gene": "UniProtKB:Q96B96",
  "term_id": "UNKNOWN:0001",
  "gene_symbol": "LDAF1",
  "gene_name": "Lipid droplet assembly factor 1"
}